{
  "gene_symbol": "PLPPR5",
  "gene_name": "Phospholipid phosphatase-related protein type 5",
  "gene": "UniProtKB:Q32ZL2",
  "term_id": "GO:0005886",
  "term_label": "plasma membrane"
}